{
  "gene_symbol": "ABCC5",
  "term_id": "GO:0140359",
  "term_label": "ABC-type transporter activity",
  "gene_name": "ATP-binding cassette sub-family C member 5",
  "gene": "UniProtKB:O15440"
}